medial membrane band [GO:0032178] (cellular component) Definition: A sterol-rich region of the plasma membrane which forms at the cell surface overlying the contractile ring and spreads into the invaginating plasma membrane surrounding the septum. References: PMID:15517003 Also known as: sterol-rich membrane band Relationships: is a type of cellular anatomical structure [GO:0110165]; is part of plasma membrane [GO:0005886]; is part of cell division site [GO:0032153]